{
  "gene": "UniProtKB:Q8N699",
  "term_id": "UNKNOWN:0002",
  "gene_name": "Myc target protein 1",
  "gene_symbol": "MYCT1",
  "term_label": "Unknown biological process"
}